{
  "gene_symbol": "MLLT3",
  "gene": "UniProtKB:P42568",
  "term_label": "positive regulation of DNA-templated transcription",
  "gene_name": "Protein AF-9",
  "term_id": "GO:0045893"
}